UGU codon-amino acid adaptor activity [GO:0033413] (MF) Sources: GOC:mah Also known as: TGT codon-amino acid adaptor activity, cysteine tRNA Note: Note that in the standard genetic code, TGT codes for cysteine. Relationships: is a type of triplet codon-amino acid adaptor activity [GO:0030533] Definition: A triplet codon-amino acid adaptor activity that recognizes a UGU codon.